{
  "gene": "UniProtKB:Q5JUR7",
  "term_label": "Unknown cellular component",
  "gene_symbol": "TEX30",
  "gene_name": "Testis-expressed protein 30",
  "term_id": "UNKNOWN:0003"
}